{
  "gene_symbol": "LRRC49",
  "term_id": "UNKNOWN:0002",
  "term_label": "Unknown biological process",
  "gene_name": "Leucine-rich repeat-containing protein 49",
  "gene": "UniProtKB:Q8IUZ0"
}